L-aspartate oxidase activity [GO:0008734] (molecular function) Relationships: is_a L-amino-acid oxidase activity [GO:0001716] Sources: EC:1.4.3.16 Also known as: L-aspartate:oxygen oxidoreductase Definition: Catalysis of the reaction: L-aspartate + O2 = iminosuccinate + H2O2. Can also use fumatate as electron acceptor under anaerobic conditions, yielding succinate.